{
  "gene_symbol": "PUM1",
  "term_label": "mRNA 3'-UTR binding",
  "gene_name": "Pumilio homolog 1",
  "term_id": "GO:0003730",
  "gene": "UniProtKB:Q14671"
}